{
  "gene_name": "Serine_threonine-protein kinase 3",
  "term_label": "positive regulation of apoptotic process",
  "gene": "UniProtKB:Q13188",
  "term_id": "GO:0043065",
  "gene_symbol": "STK3"
}